{
  "term_label": "plasma membrane",
  "gene_symbol": "EHD3",
  "gene_name": "EH domain-containing protein 3",
  "term_id": "GO:0005886",
  "gene": "UniProtKB:Q9NZN3"
}